{
  "gene": "UniProtKB:Q92698",
  "gene_name": "DNA repair and recombination protein RAD54-like",
  "gene_symbol": "RAD54L",
  "term_label": "reciprocal meiotic recombination",
  "term_id": "GO:0007131"
}